{
  "gene": "UniProtKB:P61221",
  "gene_symbol": "ABCE1",
  "gene_name": "ATP-binding cassette sub-family E member 1",
  "term_id": "GO:0005524",
  "term_label": "ATP binding"
}